{
  "term_id": "GO:0033596",
  "gene_symbol": "TBC1D7",
  "term_label": "TSC1-TSC2 complex",
  "gene": "UniProtKB:Q9P0N9",
  "gene_name": "TBC1 domain family member 7"
}